{
  "gene_name": "Probable crossover junction endonuclease EME2",
  "gene": "UniProtKB:A4GXA9",
  "gene_symbol": "EME2",
  "term_label": "resolution of meiotic recombination intermediates",
  "term_id": "GO:0000712"
}